{
  "term_id": "GO:0016324",
  "term_label": "apical plasma membrane",
  "gene_name": "Solute carrier family 15 member 1",
  "gene_symbol": "SLC15A1",
  "gene": "UniProtKB:P46059"
}